{
  "gene_name": "Protein shisa-5",
  "term_label": "Unknown molecular function",
  "gene": "UniProtKB:Q8N114",
  "gene_symbol": "SHISA5",
  "term_id": "UNKNOWN:0001"
}